negative regulation of signal transduction in absence of ligand [GO:1901099] (biological process) Subtypes: GO:2001240 Definition: Any process that stops, prevents or reduces the frequency, rate or extent of signal transduction in absence of ligand. Sources: GOC:TermGenie Relationships: is a type of negative regulation of signal transduction [GO:0009968]; negatively regulates signal transduction in absence of ligand [GO:0038034] Also known as: down regulation of non-classical signal transduction, down-regulation of non-classical signal transduction, downregulation of non-classical signal transduction, negative regulation of non-classical signal transduction, down regulation of signal transduction in absence of agonist, down regulation of signal transduction in absence of ligand, down-regulation of signal transduction in absence of agonist, down-regulation of signal transduction in absence of ligand, downregulation of signal transduction in absence of agonist, downregulation of signal transduction in absence of ligand, negative regulation of signal transduction in absence of agonist, down regulation of basal signaling, down-regulation of basal signaling, downregulation of basal signaling, inhibition of signal transduction in absence of ligand